{
  "gene": "UniProtKB:Q9HD20",
  "term_id": "GO:0055085",
  "gene_symbol": "ATP13A1",
  "gene_name": "Endoplasmic reticulum transmembrane helix translocase",
  "term_label": "transmembrane transport"
}